{
  "term_id": "UNKNOWN:0003",
  "term_label": "Unknown cellular component",
  "gene_symbol": "SMIM31",
  "gene": "UniProtKB:A0A1B0GVY4",
  "gene_name": "Small integral membrane protein 31"
}